{
  "gene": "UniProtKB:Q6ZRI6",
  "term_id": "UNKNOWN:0002",
  "gene_symbol": "C15orf39",
  "gene_name": "Uncharacterized protein C15orf39",
  "term_label": "Unknown biological process"
}